D-amino acid metabolic process [GO:0046416] (biological process) Definition: The chemical reactions and pathways involving D-amino acids, the D-enantiomers of amino acids. Sources: GOC:ai, GOC:jsg Also known as: D-amino acid metabolism Relationships: is a type of GO:0170041; is_a alpha-amino acid metabolic process [GO:1901605] Subtypes: GO:0019478, D-alanine metabolic process [GO:0046436], D-amino acid biosynthetic process [GO:0046437], D-serine metabolic process [GO:0070178], D-valine metabolic process [GO:1902114]